malonyl-CoA decarboxylase activity [GO:0050080] (molecular function) Also known as: malonyl coenzyme A decarboxylase activity, malonyl-CoA carboxy-lyase (acetyl-CoA-forming), malonyl-CoA carboxy-lyase activity Sources: EC:4.1.1.9, MetaCyc:MALONYL-COA-DECARBOXYLASE-RXN Definition: Catalysis of the reaction: malonyl-CoA = acetyl-CoA + CO2. Relationships: is a type of carboxy-lyase activity [GO:0016831]